{
  "gene": "UniProtKB:Q9BT22",
  "term_label": "mannosyltransferase activity",
  "term_id": "GO:0000030",
  "gene_symbol": "ALG1",
  "gene_name": "Chitobiosyldiphosphodolichol beta-mannosyltransferase"
}